D-leucyl-tRNA(Leu) deacylase activity [GO:0097358] (molecular function) References: PMID:10918062 Sources: GOC:se Relationships: is_a D-aminoacyl-tRNA deacylase activity [GO:0051499] Definition: Catalysis of the reaction: D-leucyl-tRNA(Leu) = D-leucine + tRNA(Leu). Removal of a D-leucine from a charged tRNA(Leu).